telogen [GO:0042639] (biological process) References: PMID:12230507 Definition: The resting phase of hair cycle. Note: Note that this term should not be used for direct annotation. If you are trying to make an annotation to x phase, it is likely that the correct annotation is 'regulation of x/y phase transition' or to a process which occurs during the reported phase. To capture the phase when a specific location or process is observed, the phase term can be used in an annotation extension (PMID:24885854) applied to a cellular component term (with the relation exists_during) or a biological process term (with the relation happens_during). Also known as: hair resting phase Relationships: is a type of GO:0044851